{
  "gene_symbol": "FHOD1",
  "term_label": "positive regulation of stress fiber assembly",
  "gene": "UniProtKB:Q9Y613",
  "term_id": "GO:0051496",
  "gene_name": "FH1_FH2 domain-containing protein 1"
}